{
  "term_id": "GO:0005886",
  "gene_name": "Activin receptor type-1C",
  "gene_symbol": "ACVR1C",
  "gene": "UniProtKB:Q8NER5",
  "term_label": "plasma membrane"
}